{
  "gene": "UniProtKB:P36897",
  "gene_symbol": "TGFBR1",
  "gene_name": "TGF-beta receptor type-1",
  "term_id": "GO:0007399",
  "term_label": "nervous system development"
}